{
  "gene_name": "Lipoyl synthase, mitochondrial",
  "term_id": "GO:0009107",
  "gene": "UniProtKB:O43766",
  "term_label": "lipoate biosynthetic process",
  "gene_symbol": "LIAS"
}